{
  "term_id": "GO:0001227",
  "gene_name": "Zinc finger protein 747",
  "gene": "UniProtKB:Q9BV97",
  "gene_symbol": "ZNF747",
  "term_label": "DNA-binding transcription repressor activity, RNA polymerase II-specific"
}